{
  "term_id": "GO:0004619",
  "gene": "UniProtKB:P18669",
  "gene_name": "Phosphoglycerate mutase 1",
  "term_label": "phosphoglycerate mutase activity",
  "gene_symbol": "PGAM1"
}